{
  "gene_name": "Mitogen-activated protein kinase kinase kinase 13",
  "term_label": "protein serine/threonine kinase activity",
  "gene": "UniProtKB:O43283",
  "gene_symbol": "MAP3K13",
  "term_id": "GO:0004674"
}